{
  "gene_name": "Zinc finger protein 121",
  "gene": "UniProtKB:P58317",
  "term_label": "regulation of transcription by RNA polymerase II",
  "gene_symbol": "ZNF121",
  "term_id": "GO:0006357"
}